{
  "gene_symbol": "NADK2",
  "gene": "UniProtKB:Q4G0N4",
  "term_label": "mitochondrion",
  "gene_name": "NAD kinase 2, mitochondrial",
  "term_id": "GO:0005739"
}